{
  "term_label": "axon",
  "term_id": "GO:0030424",
  "gene_symbol": "ROR1",
  "gene_name": "Inactive tyrosine-protein kinase transmembrane receptor ROR1",
  "gene": "UniProtKB:Q01973"
}